{
  "gene_symbol": "TRAJ22",
  "gene_name": "T cell receptor alpha joining 22 (Fragment)",
  "term_label": "Unknown biological process",
  "gene": "UniProtKB:A0A075B6Z0",
  "term_id": "UNKNOWN:0002"
}